regulation of violaceol I biosynthetic process [GO:1900713] (biological process) Subtypes: negative regulation of violaceol I biosynthetic process [GO:1900714], GO:1900715 Relationships: is a type of regulation of secondary metabolite biosynthetic process [GO:1900376]; regulates violaceol I biosynthetic process [GO:1900590] Definition: Any process that modulates the frequency, rate or extent of violaceol I biosynthetic process. Also known as: regulation of violaceol I anabolism, regulation of violaceol I biosynthesis, regulation of violaceol I formation, regulation of violaceol I synthesis Sources: GOC:TermGenie, GOC:di